muramoyltetrapeptide carboxypeptidase activity [GO:0106415] (molecular function) References: PMID:10428950, PMID:15361936 Definition: GlcNAc-MurNAc-L-alanyl-gamma-D-glutamyl-meso-diaminopimelyl-D-alanine + H2O = GlcNAc-MurNAc-L-alanyl-gamma-D-glutamyl-meso-diaminopimelate + D-alanine. Relationships: is a type of carboxypeptidase activity [GO:0004180]